{
  "gene": "UniProtKB:O75818",
  "gene_symbol": "RPP40",
  "term_label": "multimeric ribonuclease P complex",
  "gene_name": "Ribonuclease P protein subunit p40",
  "term_id": "GO:0030681"
}